UDP-glucose-glycoprotein glucose phosphotransferase activity [GO:0047358] (molecular function) Sources: EC:2.7.8.19, MetaCyc:2.7.8.19-RXN Definition: Catalysis of the reaction: glycoprotein D-mannose + UDP-D-glucose = glycoprotein 6-(D-glucose-1-phospho)-D-mannose + UMP. Relationships: is a type of GO:0016780 Also known as: Glc-phosphotransferase activity, GlcPTase activity, UDP-glucose:glycoprotein glucose-1-phosphotransferase activity, UDP-glucose:glycoprotein-D-mannose glucosephosphotransferase activity, UDPglucose-glycoprotein glucose phosphotransferase activity, UDPglucose:glycoprotein-D-mannose glucosephosphotransferase activity, uridine diphosphoglucose-glycoprotein glucose-1-phosphotransferase activity